positive regulation of myoblast fusion [GO:1901741] (biological process) References: PMID:21364645 Sources: GOC:BHF, GOC:TermGenie, GOC:rl Definition: Any process that activates or increases the frequency, rate or extent of myoblast fusion. Also known as: up regulation of myoblast fusion, up-regulation of myoblast fusion, upregulation of myoblast fusion, activation of myoblast fusion Relationships: is a type of positive regulation of syncytium formation by plasma membrane fusion [GO:0060143]; is a type of regulation of myoblast fusion [GO:1901739]; positively regulates myoblast fusion [GO:0007520]